{
  "gene_name": "Transcriptional enhancer factor TEF-4",
  "gene_symbol": "TEAD2",
  "gene": "UniProtKB:Q15562",
  "term_id": "GO:0005667",
  "term_label": "transcription regulator complex"
}